{
  "gene": "UniProtKB:Q8NGE3",
  "term_label": "olfactory receptor activity",
  "term_id": "GO:0004984",
  "gene_symbol": "OR10P1",
  "gene_name": "Olfactory receptor 10P1"
}